{
  "gene": "UniProtKB:Q4W5G0",
  "term_label": "nucleus",
  "gene_name": "Tigger transposable element-derived protein 2",
  "gene_symbol": "TIGD2",
  "term_id": "GO:0005634"
}